{
  "term_id": "GO:0005886",
  "gene_name": "Cell cycle control protein 50A",
  "gene_symbol": "TMEM30A",
  "gene": "UniProtKB:Q9NV96",
  "term_label": "plasma membrane"
}